{
  "term_label": "mitochondrial matrix",
  "term_id": "GO:0005759",
  "gene": "UniProtKB:Q9NYY8",
  "gene_symbol": "FASTKD2",
  "gene_name": "FAST kinase domain-containing protein 2, mitochondrial"
}